{
  "term_label": "plasma membrane",
  "gene_name": "Merlin",
  "gene_symbol": "NF2",
  "gene": "UniProtKB:P35240",
  "term_id": "GO:0005886"
}